{
  "gene_name": "Putative Arf-GAP with GTPase, ANK repeat and PH domain-containing protein 7",
  "term_id": "GO:0003924",
  "gene_symbol": "AGAP7P",
  "term_label": "GTPase activity",
  "gene": "UniProtKB:Q5VUJ5"
}